{
  "gene_name": "Tetratricopeptide repeat protein 24",
  "term_id": "UNKNOWN:0001",
  "gene_symbol": "TTC24",
  "term_label": "Unknown molecular function",
  "gene": "UniProtKB:A2A3L6"
}